{
  "term_id": "UNKNOWN:0003",
  "gene": "UniProtKB:Q96L94",
  "gene_name": "Sorting nexin-22",
  "gene_symbol": "SNX22",
  "term_label": "Unknown cellular component"
}